{
  "term_id": "GO:0000981",
  "gene_symbol": "PITX1",
  "term_label": "DNA-binding transcription factor activity, RNA polymerase II-specific",
  "gene": "UniProtKB:P78337",
  "gene_name": "Pituitary homeobox 1"
}